{
  "term_label": "lysophosphatidic acid acyltransferase activity",
  "gene_symbol": "LPCAT1",
  "gene_name": "Lysophosphatidylcholine acyltransferase 1",
  "gene": "UniProtKB:Q8NF37",
  "term_id": "GO:0042171"
}